cytoskeletal motor regulator activity [GO:0140659] (molecular function) Definition: Binds to and modulates the activity of a motor protein. References: PMID:23142046, PMID:33221250 Also known as: motor activity regulator activity Relationships: is a type of GO:0098772; regulates cytoskeletal motor activity [GO:0003774] Subtypes: GO:0140660, cytoskeletal motor inhibitor activity [GO:0140661]